{
  "gene_name": "Transducin-like enhancer protein 3",
  "term_label": "negative regulation of canonical Wnt signaling pathway",
  "gene_symbol": "TLE3",
  "gene": "UniProtKB:Q04726",
  "term_id": "GO:0090090"
}